{
  "term_id": "GO:0007268",
  "gene_symbol": "APBA3",
  "gene_name": "Amyloid-beta A4 precursor protein-binding family A member 3",
  "term_label": "chemical synaptic transmission",
  "gene": "UniProtKB:O96018"
}